hemangioblast cell differentiation [GO:0060217] (biological process) Definition: The process in which a relatively unspecialized cell acquires the characteristics of a mature hemangioblast. Hemangioblasts are the proposed common precursor of blood and endothelial lineages. References: PMID:15378083, PMID:9670018 Sources: GOC:bf, GOC:dph Relationships: is a type of mesodermal cell differentiation [GO:0048333]; is part of primitive hemopoiesis [GO:0060215]